{
  "gene_symbol": "LMO2",
  "term_id": "GO:0003713",
  "gene_name": "Rhombotin-2",
  "gene": "UniProtKB:P25791",
  "term_label": "transcription coactivator activity"
}